3-oxoadipyl-CoA thiolase activity [GO:0033812] (molecular function) Sources: RHEA:19481 Relationships: is a type of acetyl-CoA C-acyltransferase activity [GO:0003988] Also known as: succinyl-CoA:acetyl-CoA C-succinyltransferase activity Definition: Catalysis of the reaction: succinyl-CoA + acetyl-CoA = CoA + 3-oxoadipyl-CoA.